{
  "gene_name": "Small integral membrane protein 2",
  "term_id": "UNKNOWN:0001",
  "gene_symbol": "SMIM2",
  "gene": "UniProtKB:Q9BVW6",
  "term_label": "Unknown molecular function"
}